{
  "gene_name": "Olfactory receptor 4C3",
  "gene_symbol": "OR4C3",
  "term_id": "UNKNOWN:0002",
  "gene": "UniProtKB:Q8NH37",
  "term_label": "Unknown biological process"
}